{
  "term_label": "cytosol",
  "gene_name": "Transforming protein RhoA",
  "term_id": "GO:0005829",
  "gene": "UniProtKB:P61586",
  "gene_symbol": "RHOA"
}